{
  "gene_name": "Alpha-N-acetylneuraminide alpha-2,8-sialyltransferase",
  "term_label": "oligosaccharide metabolic process",
  "term_id": "GO:0009311",
  "gene_symbol": "ST8SIA1",
  "gene": "UniProtKB:Q92185"
}